{
  "gene_symbol": "ZNF705D",
  "gene_name": "Zinc finger protein 705D",
  "gene": "UniProtKB:P0CH99",
  "term_label": "RNA polymerase II transcription regulatory region sequence-specific DNA binding",
  "term_id": "GO:0000977"
}